{
  "term_label": "condensin complex",
  "term_id": "GO:0000796",
  "gene_name": "Condensin-2 complex subunit H2",
  "gene": "UniProtKB:Q6IBW4",
  "gene_symbol": "NCAPH2"
}